{
  "gene_symbol": "MED19",
  "gene": "UniProtKB:A0JLT2",
  "gene_name": "Mediator of RNA polymerase II transcription subunit 19",
  "term_id": "GO:0045944",
  "term_label": "positive regulation of transcription by RNA polymerase II"
}